{
  "gene": "UniProtKB:Q8N1A6",
  "term_label": "Unknown cellular component",
  "gene_name": "UPF0462 protein C4orf33",
  "gene_symbol": "C4orf33",
  "term_id": "UNKNOWN:0003"
}